{
  "gene": "UniProtKB:Q9H2W1",
  "term_label": "trans-Golgi network",
  "gene_name": "Membrane-spanning 4-domains subfamily A member 6A",
  "term_id": "GO:0005802",
  "gene_symbol": "MS4A6A"
}